{
  "term_label": "detection of chemical stimulus involved in sensory perception of smell",
  "gene": "UniProtKB:Q9H205",
  "gene_symbol": "OR2AG1",
  "term_id": "GO:0050911",
  "gene_name": "Olfactory receptor 2AG1"
}